{
  "gene_symbol": "APPL1",
  "term_label": "endosome membrane",
  "term_id": "GO:0010008",
  "gene": "UniProtKB:Q9UKG1",
  "gene_name": "DCC-interacting protein 13-alpha"
}